{
  "term_id": "GO:0042147",
  "gene_symbol": "TMEM87B",
  "gene_name": "Transmembrane protein 87B",
  "gene": "UniProtKB:Q96K49",
  "term_label": "retrograde transport, endosome to Golgi"
}